{
  "gene_name": "Lutropin subunit beta",
  "gene": "UniProtKB:P01229",
  "term_label": "ovarian follicle development",
  "term_id": "GO:0001541",
  "gene_symbol": "LHB"
}